{
  "gene_name": "BTB_POZ domain-containing protein KCTD12",
  "gene_symbol": "KCTD12",
  "gene": "UniProtKB:Q96CX2",
  "term_label": "presynaptic membrane",
  "term_id": "GO:0042734"
}